{
  "gene": "UniProtKB:Q8IXL9",
  "gene_name": "IQ domain-containing protein F2",
  "gene_symbol": "IQCF2",
  "term_id": "UNKNOWN:0003",
  "term_label": "Unknown cellular component"
}